{
  "gene_name": "G1_S-specific cyclin-D2",
  "gene": "UniProtKB:P30279",
  "term_id": "GO:0000082",
  "gene_symbol": "CCND2",
  "term_label": "G1/S transition of mitotic cell cycle"
}